formation of primary germ layer [GO:0001704] (biological process) Relationships: is a type of GO:0048646; is part of gastrulation [GO:0007369] Definition: The formation of the ectoderm, mesoderm and endoderm during gastrulation. Sources: GOC:go_curators Subtypes: GO:0001705, GO:0001706, GO:0001707